{
  "gene": "UniProtKB:P30520",
  "term_id": "GO:0005737",
  "gene_name": "Adenylosuccinate synthetase isozyme 2",
  "term_label": "cytoplasm",
  "gene_symbol": "ADSS2"
}